{
  "term_id": "GO:0005509",
  "gene_name": "Regucalcin",
  "term_label": "calcium ion binding",
  "gene_symbol": "RGN",
  "gene": "UniProtKB:Q15493"
}